{
  "term_label": "protein disulfide isomerase activity",
  "gene_symbol": "PDIA3",
  "gene_name": "Protein disulfide-isomerase A3",
  "gene": "UniProtKB:P30101",
  "term_id": "GO:0003756"
}